{
  "gene_symbol": "MASP1",
  "term_id": "GO:0001867",
  "gene_name": "Mannan-binding lectin serine protease 1",
  "term_label": "complement activation, lectin pathway",
  "gene": "UniProtKB:P48740"
}